cardiac Troponin complex [GO:1990584] (cellular component) Definition: A complex of accessory proteins (cardiac troponin T, cardiac troponin I and cardiac troponin C) found associated with actin in cardiac muscle thin filaments; involved in calcium regulation important for muscle contraction. References: PMID:12840750 Sources: GOC:ame Relationships: is a type of troponin complex [GO:0005861] Also known as: cTnC:cTnI:cTnT